{
  "gene_name": "Protein reprimo",
  "gene": "UniProtKB:Q9NS64",
  "term_id": "GO:0005737",
  "term_label": "cytoplasm",
  "gene_symbol": "RPRM"
}